{
  "gene_symbol": "MYH11",
  "gene_name": "Myosin-11",
  "term_label": "actin filament binding",
  "gene": "UniProtKB:P35749",
  "term_id": "GO:0051015"
}